{
  "term_label": "regulation of transcription by RNA polymerase II",
  "term_id": "GO:0006357",
  "gene_name": "Transcription factor 21",
  "gene": "UniProtKB:O43680",
  "gene_symbol": "TCF21"
}